{
  "gene": "UniProtKB:A6NFK2",
  "term_id": "GO:0120044",
  "term_label": "stereocilium base",
  "gene_name": "Glutaredoxin domain-containing cysteine-rich protein 2",
  "gene_symbol": "GRXCR2"
}